negative regulation of mitochondrial translation [GO:0070130] (biological process) Definition: Any process that stops, prevents, or reduces the frequency, rate or extent of the chemical reactions and pathways resulting in the formation of proteins by the translation of mRNA in a mitochondrion. Also known as: negative regulation of mitochondrial protein anabolism, negative regulation of mitochondrial protein biosynthesis, negative regulation of mitochondrial protein formation, negative regulation of mitochondrial protein synthesis Subtypes: negative regulation of mitochondrial translational elongation [GO:1905083] Sources: GOC:mah Relationships: is a type of negative regulation of translation [GO:0017148]; is a type of regulation of mitochondrial translation [GO:0070129]; negatively regulates mitochondrial translation [GO:0032543]